{
  "term_id": "GO:0005737",
  "gene_symbol": "HSPB6",
  "term_label": "cytoplasm",
  "gene_name": "Heat shock protein beta-6",
  "gene": "UniProtKB:O14558"
}